{
  "gene": "UniProtKB:P16050",
  "term_id": "GO:0004052",
  "gene_name": "Polyunsaturated fatty acid lipoxygenase ALOX15",
  "gene_symbol": "ALOX15",
  "term_label": "arachidonate 12(S)-lipoxygenase activity"
}